{
  "gene_symbol": "DPAGT1",
  "term_id": "GO:0016020",
  "term_label": "membrane",
  "gene": "UniProtKB:Q9H3H5",
  "gene_name": "UDP-N-acetylglucosamine--dolichyl-phosphate N-acetylglucosaminephosphotransferase"
}